{
  "gene": "UniProtKB:Q12830",
  "term_label": "Unknown molecular function",
  "term_id": "UNKNOWN:0001",
  "gene_name": "Nucleosome-remodeling factor subunit BPTF",
  "gene_symbol": "BPTF"
}